negative regulation of Atg1/ULK1 kinase complex assembly [GO:1905865] (biological process) Definition: Any process that stops, prevents or reduces the frequency, rate or extent of Atg1/ULK1 kinase complex assembly. References: PMID:26567215 Sources: GOC:TermGenie, GOC:autophagy, GOC:mf, GO_REF:0000058 Relationships: is a type of GO:0031333; is a type of regulation of Atg1/ULK1 kinase complex assembly [GO:1905864]; negatively regulates Atg1/ULK1 kinase complex assembly [GO:1904745] Also known as: down regulation of ATG1 kinase complex assembly, down regulation of ATG1 kinase complex formation, down regulation of ATG1-ATG13 complex assembly, down regulation of ATG1-ATG13 complex formation, down regulation of ATG1/ULK1 kinase complex assembly, down regulation of ATG1/ULK1 kinase complex formation, down regulation of ATG1/ULK1 signaling complex assembly, down regulation of ATG1/ULK1 signaling complex formation, down regulation of Atg1p signalling complex assembly, down regulation of Atg1p signalling complex formation, down regulation of ULK1 signaling complex assembly, down regulation of ULK1 signaling complex formation, down regulation of ULK1-ATG13-FIP200 complex assembly, down regulation of ULK1-ATG13-FIP200 complex formation, down regulation of ULK1-ATG13-RB1CC1 complex assembly, down regulation of ULK1-ATG13-RB1CC1 complex formation, down-regulation of ATG1 kinase complex assembly, down-regulation of ATG1 kinase complex formation, down-regulation of ATG1-ATG13 complex assembly, down-regulation of ATG1-ATG13 complex formation, down-regulation of ATG1/ULK1 kinase complex assembly, down-regulation of ATG1/ULK1 kinase complex formation, down-regulation of ATG1/ULK1 signaling complex assembly, down-regulation of ATG1/ULK1 signaling complex formation, down-regulation of Atg1p signalling complex assembly, down-regulation of Atg1p signalling complex formation, down-regulation of ULK1 signaling complex assembly, down-regulation of ULK1 signaling complex formation, down-regulation of ULK1-ATG13-FIP200 complex assembly, down-regulation of ULK1-ATG13-FIP200 complex formation, down-regulation of ULK1-ATG13-RB1CC1 complex assembly, down-regulation of ULK1-ATG13-RB1CC1 complex formation, downregulation of ATG1 kinase complex assembly, downregulation of ATG1 kinase complex formation, downregulation of ATG1-ATG13 complex assembly, downregulation of ATG1-ATG13 complex formation, downregulation of ATG1/ULK1 kinase complex assembly, downregulation of ATG1/ULK1 kinase complex formation, downregulation of ATG1/ULK1 signaling complex assembly, downregulation of ATG1/ULK1 signaling complex formation, downregulation of Atg1p signalling complex assembly, downregulation of Atg1p signalling complex formation, downregulation of ULK1 signaling complex assembly, downregulation of ULK1 signaling complex formation, downregulation of ULK1-ATG13-FIP200 complex assembly, downregulation of ULK1-ATG13-FIP200 complex formation, downregulation of ULK1-ATG13-RB1CC1 complex assembly, downregulation of ULK1-ATG13-RB1CC1 complex formation, negative regulation of ATG1 kinase complex assembly, negative regulation of ATG1 kinase complex formation, negative regulation of ATG1-ATG13 complex assembly, negative regulation of ATG1-ATG13 complex formation, negative regulation of ATG1/ULK1 kinase complex formation, negative regulation of ATG1/ULK1 signaling complex assembly, negative regulation of ATG1/ULK1 signaling complex formation, negative regulation of Atg1p signalling complex assembly, negative regulation of Atg1p signalling complex formation, negative regulation of ULK1 signaling complex assembly, negative regulation of ULK1 signaling complex formation, negative regulation of ULK1-ATG13-FIP200 complex assembly, negative regulation of ULK1-ATG13-FIP200 complex formation, negative regulation of ULK1-ATG13-RB1CC1 complex assembly, negative regulation of ULK1-ATG13-RB1CC1 complex formation, inhibition of ATG1 kinase complex assembly, inhibition of ATG1 kinase complex formation, inhibition of ATG1-ATG13 complex assembly, inhibition of ATG1-ATG13 complex formation, inhibition of ATG1/ULK1 kinase complex assembly, inhibition of ATG1/ULK1 kinase complex formation, inhibition of ATG1/ULK1 signaling complex assembly, inhibition of ATG1/ULK1 signaling complex formation, inhibition of Atg1p signalling complex assembly, inhibition of Atg1p signalling complex formation, inhibition of ULK1 signaling complex assembly, inhibition of ULK1 signaling complex formation, inhibition of ULK1-ATG13-FIP200 complex assembly, inhibition of ULK1-ATG13-FIP200 complex formation, inhibition of ULK1-ATG13-RB1CC1 complex assembly, inhibition of ULK1-ATG13-RB1CC1 complex formation